{
  "term_label": "Unknown cellular component",
  "gene_symbol": "NPDC1",
  "gene_name": "Neural proliferation differentiation and control protein 1",
  "gene": "UniProtKB:Q9NQX5",
  "term_id": "UNKNOWN:0003"
}